positive regulation of locomotor rhythm [GO:1904061] (biological process) References: PMID:16310969 Sources: GOC:TermGenie, GO_REF:0000058 Definition: Any process that activates or increases the frequency, rate or extent of locomotor rhythm. Relationships: is a type of positive regulation of circadian rhythm [GO:0042753]; is_a positive regulation of behavior [GO:0048520]; is a type of regulation of locomotor rhythm [GO:1904059]; positively regulates locomotor rhythm [GO:0045475] Also known as: up regulation of locomotor rhythm, up-regulation of locomotor rhythm, upregulation of locomotor rhythm, activation of circadian locomotor activity rhythm, activation of locomotor rhythm, positive regulation of circadian locomotor activity rhythm, up regulation of circadian locomotor activity rhythm, up-regulation of circadian locomotor activity rhythm, upregulation of circadian locomotor activity rhythm